{
  "term_id": "UNKNOWN:0001",
  "gene": "UniProtKB:I3L0S3",
  "gene_name": "Putative uncharacterized protein PYCARD-AS1",
  "term_label": "Unknown molecular function",
  "gene_symbol": "PYCARD-AS1"
}